{
  "term_id": "GO:1902711",
  "term_label": "GABA-A receptor complex",
  "gene_name": "Gamma-aminobutyric acid receptor subunit rho-3",
  "gene_symbol": "GABRR3",
  "gene": "UniProtKB:A8MPY1"
}